{
  "term_id": "GO:0001725",
  "term_label": "stress fiber",
  "gene_name": "Alpha-actinin-1",
  "gene": "UniProtKB:P12814",
  "gene_symbol": "ACTN1"
}